{
  "term_label": "extracellular space",
  "gene": "UniProtKB:P0DN87",
  "gene_name": "Choriogonadotropin subunit beta 7",
  "term_id": "GO:0005615",
  "gene_symbol": "CGB7"
}